{
  "term_label": "methionine adenosyltransferase complex",
  "gene_symbol": "MAT2B",
  "gene_name": "Methionine adenosyltransferase 2 subunit beta",
  "gene": "UniProtKB:Q9NZL9",
  "term_id": "GO:0048269"
}